{
  "gene_symbol": "PLEKHG3",
  "term_id": "GO:2000114",
  "gene": "UniProtKB:A1L390",
  "gene_name": "Pleckstrin homology domain-containing family G member 3",
  "term_label": "regulation of establishment of cell polarity"
}